{
  "gene_name": "Sodium-dependent multivitamin transporter",
  "gene_symbol": "SLC5A6",
  "term_label": "Unknown cellular component",
  "gene": "UniProtKB:Q9Y289",
  "term_id": "UNKNOWN:0003"
}